{
  "term_id": "GO:0005615",
  "gene_symbol": "SFTPA2",
  "gene_name": "Pulmonary surfactant-associated protein A2",
  "term_label": "extracellular space",
  "gene": "UniProtKB:Q8IWL1"
}